{
  "term_label": "plasma membrane",
  "gene_symbol": "GPR151",
  "gene_name": "G-protein coupled receptor 151",
  "term_id": "GO:0005886",
  "gene": "UniProtKB:Q8TDV0"
}